box H/ACA snoRNP complex binding [GO:0062065] (molecular function) References: PMID:10679015 Relationships: is_a snoRNP binding [GO:0030519] Definition: Binding to a box H/ACA snoRNP complex.